negative regulation of calcium ion transmembrane transport [GO:1903170] (biological process) Note: human HRC regulates RYR2 and thus regulates transmembrane transport of calcium from SR to cytosol Relationships: is a type of negative regulation of calcium ion transport [GO:0051926]; is a type of regulation of calcium ion transmembrane transport [GO:1903169]; is a type of negative regulation of cation transmembrane transport [GO:1904063]; negatively regulates calcium ion transmembrane transport [GO:0070588] Subtypes: negative regulation of calcium ion transport into cytosol [GO:0010523], negative regulation of release of sequestered calcium ion into cytosol [GO:0051280], negative regulation of calcium import into the mitochondrion [GO:0110099], negative regulation of calcium ion transmembrane transporter activity [GO:1901020], negative regulation of calcium ion transmembrane transport via high voltage-gated calcium channel [GO:1904878], negative regulation of calcium ion export across plasma membrane [GO:1905913], GO:1905949 References: PMID:24125847 Sources: GOC:BHF, GOC:TermGenie, GOC:rl, GO_REF:0000058 Definition: Any process that stops, prevents or reduces the frequency, rate or extent of calcium ion transmembrane transport. Also known as: down regulation of calcium ion membrane transport, down regulation of calcium ion transmembrane transport, down regulation of transmembrane calcium transport, down-regulation of calcium ion membrane transport, down-regulation of calcium ion transmembrane transport, down-regulation of transmembrane calcium transport, downregulation of calcium ion membrane transport, downregulation of calcium ion transmembrane transport, downregulation of transmembrane calcium transport, negative regulation of calcium ion membrane transport, negative regulation of transmembrane calcium transport, inhibition of calcium ion membrane transport, inhibition of calcium ion transmembrane transport, inhibition of transmembrane calcium transport